{
  "term_id": "GO:0017157",
  "gene_name": "Leucine-rich repeat LGI family member 3",
  "term_label": "regulation of exocytosis",
  "gene": "UniProtKB:Q8N145",
  "gene_symbol": "LGI3"
}